{
  "gene": "UniProtKB:Q9Y5Y4",
  "term_label": "neuropeptide signaling pathway",
  "gene_name": "Prostaglandin D2 receptor 2",
  "gene_symbol": "PTGDR2",
  "term_id": "GO:0007218"
}